{
  "gene_symbol": "SPEM3",
  "term_label": "cytoplasm",
  "gene_name": "Uncharacterized protein SPEM3",
  "gene": "UniProtKB:A0A1B0GUW6",
  "term_id": "GO:0005737"
}